viral inner capsid [GO:0039625] (cellular component) Definition: The inner layer of a double or triple concentric icosahedral capsid. Inner capsids are part of reoviridae and cystoviridae virions. Sources: UniProtKB-KW:KW-1153 Relationships: is a type of virion component [GO:0044423]; is part of icosahedral viral capsid [GO:0019030] Also known as: inner capsid